{
  "term_label": "late endosome membrane",
  "gene": "UniProtKB:Q5T0T0",
  "gene_name": "E3 ubiquitin-protein ligase MARCHF8",
  "term_id": "GO:0031902",
  "gene_symbol": "MARCHF8"
}